{
  "gene": "UniProtKB:Q8N8Q1",
  "gene_name": "Probable transmembrane reductase CYB561D1",
  "gene_symbol": "CYB561D1",
  "term_label": "endoplasmic reticulum membrane",
  "term_id": "GO:0005789"
}